{
  "gene_name": "Prospero homeobox protein 2",
  "gene_symbol": "PROX2",
  "term_id": "GO:0000981",
  "term_label": "DNA-binding transcription factor activity, RNA polymerase II-specific",
  "gene": "UniProtKB:Q3B8N5"
}